{
  "term_id": "GO:0006814",
  "gene_name": "Sodium-dependent multivitamin transporter",
  "gene": "UniProtKB:Q9Y289",
  "term_label": "sodium ion transport",
  "gene_symbol": "SLC5A6"
}